L-amino acid biosynthetic process [GO:0170034] (biological process) Definition: The chemical reactions and pathways resulting in the formation of L-amino acids, the L-enantiomers of amino acids. Also known as: L-amino acid anabolism, L-amino acid biosynthesis, L-amino acid formation, L-amino acid synthesis Subtypes: L-histidine biosynthetic process [GO:0000105], GO:0000162, GO:0006564, L-tyrosine biosynthetic process [GO:0006571], aspartate family amino acid biosynthetic process [GO:0009067], pyruvate family amino acid biosynthetic process [GO:0009079], GO:0009084, L-phenylalanine biosynthetic process [GO:0009094], L-proline betaine biosynthetic process [GO:0019503], GO:0034268, GO:0046312, L-beta-ethynylserine biosynthetic process [GO:0062142], L-propargylglycine biosynthetic process [GO:0062143], GO:0071269, GO:1903185, 3-cyano-L-alanine biosynthetic process [GO:1903560] Sources: GOC:edw Relationships: is a type of GO:0170033; is a type of GO:1901607